regulation of endopeptidase activity [GO:0052548] (biological process) Subtypes: positive regulation of endopeptidase activity [GO:0010950], negative regulation of endopeptidase activity [GO:0010951], GO:1900003 Relationships: is a type of regulation of peptidase activity [GO:0052547]; regulates endopeptidase activity [GO:0004175] Definition: Any process that modulates the frequency, rate or extent of endopeptidase activity, the endohydrolysis of peptide bonds within proteins. Also known as: protease regulator activity Sources: GOC:ai, GOC:hjd